{
  "term_label": "GTP binding",
  "gene": "UniProtKB:Q9HB90",
  "gene_symbol": "RRAGC",
  "term_id": "GO:0005525",
  "gene_name": "Ras-related GTP-binding protein C"
}